regulation of developmental vegetative growth [GO:1905613] (BP) References: PMID:11606552 Sources: GOC:TermGenie, GO_REF:0000058 Definition: Any process that modulates the frequency, rate or extent of developmental vegetative growth. Relationships: is_a regulation of developmental growth [GO:0048638]; regulates developmental vegetative growth [GO:0080186] Subtypes: regulation of vegetative meristem growth [GO:0010083], negative regulation of developmental vegetative growth [GO:1905614], positive regulation of developmental vegetative growth [GO:1905615]